{
  "gene_symbol": "IGF1",
  "term_label": "extracellular space",
  "term_id": "GO:0005615",
  "gene": "UniProtKB:P05019",
  "gene_name": "Insulin-like growth factor I"
}